side of membrane [GO:0098552] (CC) Sources: GOC:dos Relationships: is a type of GO:0110165; is part of GO:0016020; has part leaflet of membrane bilayer [GO:0097478] Subtypes: GO:0009897, external side of cell outer membrane [GO:0031240], periplasmic side of cell outer membrane [GO:0031241], GO:0098562, GO:0098569, stromal side of plastid inner membrane [GO:0098570], lumenal side of plastid thylakoid membrane [GO:0098571], stromal side of plastid thylakoid membrane [GO:0098572], lumenal side of membrane [GO:0098576] Definition: A cellular component consisting of one leaflet of a membrane bilayer and any proteins embedded or anchored in it or attached to its surface.